{
  "term_label": "Unknown cellular component",
  "gene_name": "Putative KRAB domain-containing protein ZNF788",
  "gene": "UniProtKB:Q6ZQV5",
  "gene_symbol": "ZNF788P",
  "term_id": "UNKNOWN:0003"
}